{
  "gene_name": "U5 small nuclear ribonucleoprotein TSSC4",
  "term_label": "U5 snRNP",
  "gene_symbol": "TSSC4",
  "gene": "UniProtKB:Q9Y5U2",
  "term_id": "GO:0005682"
}